{
  "gene_name": "Cartilage matrix protein",
  "term_label": "extracellular matrix",
  "gene_symbol": "MATN1",
  "gene": "UniProtKB:P21941",
  "term_id": "GO:0031012"
}